{
  "term_label": "Unknown molecular function",
  "gene": "UniProtKB:Q6ICL3",
  "gene_name": "Transport and Golgi organization protein 2 homolog",
  "gene_symbol": "TANGO2",
  "term_id": "UNKNOWN:0001"
}